acetaldehyde dehydrogenase (NADP+) activity [GO:0140088] (molecular function) Relationships: is a type of aldehyde dehydrogenase (NADP+) activity [GO:0033721] Definition: Catalysis of the reaction: acetaldehyde + NADP+ + H2O = acetate + NADPH + 2 H+. References: PMID:15659684, PMID:9473035 Sources: RHEA:25298